{
  "term_id": "GO:0000978",
  "gene": "UniProtKB:Q9ULX9",
  "gene_symbol": "MAFF",
  "term_label": "RNA polymerase II cis-regulatory region sequence-specific DNA binding",
  "gene_name": "Transcription factor MafF"
}